{
  "gene_name": "Relaxin-3 receptor 2",
  "term_id": "GO:0007218",
  "gene": "UniProtKB:Q8TDU9",
  "gene_symbol": "RXFP4",
  "term_label": "neuropeptide signaling pathway"
}